{
  "gene_symbol": "GPR45",
  "gene_name": "Probable G-protein coupled receptor 45",
  "term_label": "G protein-coupled receptor signaling pathway",
  "term_id": "GO:0007186",
  "gene": "UniProtKB:Q9Y5Y3"
}